{
  "gene_symbol": "NUP88",
  "term_id": "GO:0005643",
  "term_label": "nuclear pore",
  "gene_name": "Nuclear pore complex protein Nup88",
  "gene": "UniProtKB:Q99567"
}